proteasome complex [GO:0000502] (cellular component) Definition: A large multisubunit complex which catalyzes protein degradation, found in eukaryotes, archaea and some bacteria. In eukaryotes, this complex consists of the barrel shaped proteasome core complex and one or two associated proteins or complexes that act in regulating entry into or exit from the core. Also known as: proteasome, 26S proteasome Relationships: is a type of intracellular protein-containing complex [GO:0140535]; is a type of endopeptidase complex [GO:1905369] Subtypes: nuclear proteasome complex [GO:0031595], cytosolic proteasome complex [GO:0031597], spermatoproteasome complex [GO:1990111] Sources: GOC:rb, Wikipedia:Proteasome